{
  "gene_symbol": "CCR2",
  "gene_name": "C-C chemokine receptor type 2",
  "term_label": "external side of plasma membrane",
  "gene": "UniProtKB:P41597",
  "term_id": "GO:0009897"
}